{
  "gene_symbol": "PRMT7",
  "term_label": "Unknown cellular component",
  "gene_name": "Protein arginine N-methyltransferase 7",
  "term_id": "UNKNOWN:0003",
  "gene": "UniProtKB:Q9NVM4"
}